{
  "term_label": "Unknown biological process",
  "gene_name": "Putative ankyrin repeat domain-containing protein 30B-like",
  "gene": "UniProtKB:A7E2S9",
  "term_id": "UNKNOWN:0002",
  "gene_symbol": "ANKRD30BL"
}